{
  "term_label": "Unknown molecular function",
  "gene_name": "Centrosomal protein 43",
  "gene": "UniProtKB:O95684",
  "term_id": "UNKNOWN:0001",
  "gene_symbol": "CEP43"
}